{
  "term_id": "GO:0006355",
  "gene": "UniProtKB:P10075",
  "gene_name": "Zinc finger protein GLI4",
  "term_label": "regulation of DNA-templated transcription",
  "gene_symbol": "GLI4"
}